{
  "gene_name": "TBC1 domain family member 3I",
  "gene": "UniProtKB:A0A087WXS9",
  "term_label": "Unknown cellular component",
  "gene_symbol": "TBC1D3I",
  "term_id": "UNKNOWN:0003"
}